{
  "term_label": "regulation of apoptotic process",
  "gene_name": "Ubiquitin carboxyl-terminal hydrolase 17-like protein 20",
  "gene_symbol": "USP17L20",
  "term_id": "GO:0042981",
  "gene": "UniProtKB:D6RJB6"
}